{
  "gene": "UniProtKB:Q9BQ15",
  "term_id": "GO:0000724",
  "gene_symbol": "NABP2",
  "term_label": "double-strand break repair via homologous recombination",
  "gene_name": "SOSS complex subunit B1"
}